{
  "gene_symbol": "BCORL1",
  "term_label": "negative regulation of transcription by RNA polymerase II",
  "gene_name": "BCL-6 corepressor-like protein 1",
  "gene": "UniProtKB:Q5H9F3",
  "term_id": "GO:0000122"
}